{
  "term_label": "acetyl-CoA biosynthetic process",
  "term_id": "GO:0006085",
  "gene_name": "Malonyl-CoA decarboxylase, mitochondrial",
  "gene": "UniProtKB:O95822",
  "gene_symbol": "MLYCD"
}